EKC/KEOPS complex [GO:0000408] (CC) Relationships: is a type of transferase complex [GO:1990234] Definition: A protein complex involved in t6A tRNA modification. For example, in Saccharomyces cerevisiae the complex contains Bud32p, Kae1p, Gon7p, Cgi121p, and Pcc1p. Note: Originally proposed to be involved in transcription as well as promoting telomere uncapping and telomere elongation. Also known as: KEOPS/EKC complex, endopeptidase-like kinase chromatin-associated protein complex, kinase, putative endopeptidase and other proteins of small size protein complex, TCTC, threonyl-carbamoly transferase complex References: PMID:16564010, PMID:16874308, PMID:21183954, PMID:23945934 Sources: GOC:elh, GOC:vw